L-leucine 2,3-aminomutase activity [GO:0050047] (molecular function) Sources: RHEA:10284 Definition: Catalysis of the reaction: L-leucine = (3R)-beta-leucine. Relationships: is a type of intramolecular aminotransferase activity [GO:0016869] Also known as: (2S)-alpha-leucine 2,3-aminomutase activity, leucine 2,3-aminomutase activity